primary sex determination, germ-line [GO:0007542] (biological process) Relationships: is a type of GO:0007538; is part of germ-line sex determination [GO:0018992] Sources: GOC:ems Subtypes: GO:0019099, male germ-line sex determination [GO:0019100] Definition: The transmission of information about sexual status, from the initial general determination, to signals specific to the germ-line.